{
  "term_label": "Set1C/COMPASS complex",
  "gene_name": "CXXC-type zinc finger protein 1",
  "gene_symbol": "CXXC1",
  "gene": "UniProtKB:Q9P0U4",
  "term_id": "GO:0048188"
}